{
  "term_label": "positive regulation of MAPK cascade",
  "gene": "UniProtKB:P07550",
  "gene_symbol": "ADRB2",
  "gene_name": "Beta-2 adrenergic receptor",
  "term_id": "GO:0043410"
}